positive regulation of epidermal growth factor receptor signaling pathway involved in heart process [GO:1905284] (biological process) Relationships: is a type of positive regulation of epidermal growth factor receptor signaling pathway [GO:0045742]; is a type of positive regulation of multicellular organismal process [GO:0051240]; is a type of regulation of epidermal growth factor receptor signaling pathway involved in heart process [GO:1905282]; positively regulates GO:1905251 References: PMID:23069713 Sources: GOC:BHF, GOC:BHF_miRNA, GOC:TermGenie, GOC:bc, GO_REF:0000058 Definition: Any process that activates or increases the frequency, rate or extent of epidermal growth factor receptor signaling pathway involved in heart process. Also known as: positive regulation of EGF receptor signaling pathway involved in heart process, positive regulation of EGF receptor signalling pathway involved in heart process, positive regulation of EGFR signaling pathway involved in heart process, positive regulation of ERBB1 signaling pathway involved in heart process, positive regulation of epidermal growth factor receptor signalling pathway involved in heart process, positive regulation of receptor tyrosine-protein kinase erbB-1 signaling pathway involved in heart process, up regulation of EGF receptor signaling pathway involved in heart process, up regulation of EGF receptor signalling pathway involved in heart process, up regulation of EGFR signaling pathway involved in heart process, up regulation of ERBB1 signaling pathway involved in heart process, up regulation of epidermal growth factor receptor signaling pathway involved in heart process, up regulation of epidermal growth factor receptor signalling pathway involved in heart process, up regulation of receptor tyrosine-protein kinase erbB-1 signaling pathway involved in heart process, up-regulation of EGF receptor signaling pathway involved in heart process, up-regulation of EGF receptor signalling pathway involved in heart process, up-regulation of EGFR signaling pathway involved in heart process, up-regulation of ERBB1 signaling pathway involved in heart process, up-regulation of epidermal growth factor receptor signaling pathway involved in heart process, up-regulation of epidermal growth factor receptor signalling pathway involved in heart process, up-regulation of receptor tyrosine-protein kinase erbB-1 signaling pathway involved in heart process, upregulation of EGF receptor signaling pathway involved in heart process, upregulation of EGF receptor signalling pathway involved in heart process, upregulation of EGFR signaling pathway involved in heart process, upregulation of ERBB1 signaling pathway involved in heart process, upregulation of epidermal growth factor receptor signaling pathway involved in heart process, upregulation of epidermal growth factor receptor signalling pathway involved in heart process, upregulation of receptor tyrosine-protein kinase erbB-1 signaling pathway involved in heart process, activation of EGF receptor signaling pathway involved in heart process, activation of EGF receptor signalling pathway involved in heart process, activation of EGFR signaling pathway involved in heart process, activation of ERBB1 signaling pathway involved in heart process, activation of epidermal growth factor receptor signaling pathway involved in heart process, activation of epidermal growth factor receptor signalling pathway involved in heart process, activation of receptor tyrosine-protein kinase erbB-1 signaling pathway involved in heart process, activation of EGF receptor signaling pathway involved in cardiac process, activation of EGF receptor signalling pathway involved in cardiac process, activation of EGFR signaling pathway involved in cardiac process, activation of ERBB1 signaling pathway involved in cardiac process, activation of epidermal growth factor receptor signaling pathway involved in cardiac process, activation of epidermal growth factor receptor signalling pathway involved in cardiac process, activation of receptor tyrosine-protein kinase erbB-1 signaling pathway involved in cardiac process, positive regulation of EGF receptor signaling pathway involved in cardiac process, positive regulation of EGF receptor signalling pathway involved in cardiac process, positive regulation of EGFR signaling pathway involved in cardiac process, positive regulation of ERBB1 signaling pathway involved in cardiac process, positive regulation of epidermal growth factor receptor signaling pathway involved in cardiac process, positive regulation of epidermal growth factor receptor signalling pathway involved in cardiac process, positive regulation of receptor tyrosine-protein kinase erbB-1 signaling pathway involved in cardiac process, up regulation of EGF receptor signaling pathway involved in cardiac process, up regulation of EGF receptor signalling pathway involved in cardiac process, up regulation of EGFR signaling pathway involved in cardiac process, up regulation of ERBB1 signaling pathway involved in cardiac process, up regulation of epidermal growth factor receptor signaling pathway involved in cardiac process, up regulation of epidermal growth factor receptor signalling pathway involved in cardiac process, up regulation of receptor tyrosine-protein kinase erbB-1 signaling pathway involved in cardiac process, up-regulation of EGF receptor signaling pathway involved in cardiac process, up-regulation of EGF receptor signalling pathway involved in cardiac process, up-regulation of EGFR signaling pathway involved in cardiac process, up-regulation of ERBB1 signaling pathway involved in cardiac process, up-regulation of epidermal growth factor receptor signaling pathway involved in cardiac process, up-regulation of epidermal growth factor receptor signalling pathway involved in cardiac process, up-regulation of receptor tyrosine-protein kinase erbB-1 signaling pathway involved in cardiac process, upregulation of EGF receptor signaling pathway involved in cardiac process, upregulation of EGF receptor signalling pathway involved in cardiac process, upregulation of EGFR signaling pathway involved in cardiac process, upregulation of ERBB1 signaling pathway involved in cardiac process, upregulation of epidermal growth factor receptor signaling pathway involved in cardiac process, upregulation of epidermal growth factor receptor signalling pathway involved in cardiac process, upregulation of receptor tyrosine-protein kinase erbB-1 signaling pathway involved in cardiac process